negative regulation of nitric oxide-cGMP mediated signal transduction [GO:0141151] (BP) Definition: Any process that decreases the rate, frequency or extent of nitric oxide-cGMP mediated signal transduction. Relationships: is a type of negative regulation of nitric oxide mediated signal transduction [GO:0010751]; is a type of regulation of nitric oxide-cGMP mediated signal transduction [GO:0141149]; negatively regulates nitric oxide-cGMP-mediated signaling [GO:0038060] References: PMID:35931019